{
  "gene_name": "Unconventional myosin-VI",
  "gene": "UniProtKB:Q9UM54",
  "term_label": "actin filament organization",
  "gene_symbol": "MYO6",
  "term_id": "GO:0007015"
}